{
  "gene_symbol": "MAPK8",
  "gene": "UniProtKB:P45983",
  "term_id": "GO:0043065",
  "term_label": "positive regulation of apoptotic process",
  "gene_name": "Mitogen-activated protein kinase 8"
}